{
  "gene_symbol": "TMLHE",
  "term_id": "GO:0005739",
  "term_label": "mitochondrion",
  "gene": "UniProtKB:Q9NVH6",
  "gene_name": "Trimethyllysine dioxygenase, mitochondrial"
}